{
  "term_id": "UNKNOWN:0001",
  "term_label": "Unknown molecular function",
  "gene": "UniProtKB:Q3LI81",
  "gene_name": "Keratin-associated protein 27-1",
  "gene_symbol": "KRTAP27-1"
}